{
  "gene_symbol": "F7",
  "gene_name": "Coagulation factor VII",
  "gene": "UniProtKB:P08709",
  "term_label": "protein processing",
  "term_id": "GO:0016485"
}